{
  "gene_symbol": "ZMIZ2",
  "gene_name": "Zinc finger MIZ domain-containing protein 2",
  "gene": "UniProtKB:Q8NF64",
  "term_label": "transcription coactivator activity",
  "term_id": "GO:0003713"
}